dTMP metabolic process [GO:0046073] (biological process) Subtypes: GO:0006231, dTMP catabolic process [GO:0046074] Definition: The chemical reactions and pathways involving dTMP, deoxyribosylthymine monophosphate (2'-deoxyribosylthymine 5'-phosphate). Relationships: is a type of GO:0009176; is a type of pyrimidine deoxyribonucleotide metabolic process [GO:0009219] Sources: GOC:go_curators Also known as: dTMP metabolism